{
  "gene_symbol": "OPRK1",
  "gene_name": "Kappa-type opioid receptor",
  "term_label": "G protein-coupled opioid receptor signaling pathway",
  "gene": "UniProtKB:P41145",
  "term_id": "GO:0038003"
}